{
  "term_id": "GO:0006886",
  "gene_symbol": "STX2",
  "term_label": "intracellular protein transport",
  "gene": "UniProtKB:P32856",
  "gene_name": "Syntaxin-2"
}